{
  "gene": "UniProtKB:O00571",
  "gene_symbol": "DDX3X",
  "term_id": "GO:0010629",
  "term_label": "negative regulation of gene expression",
  "gene_name": "ATP-dependent RNA helicase DDX3X"
}